{
  "gene": "UniProtKB:P01614",
  "term_id": "UNKNOWN:0001",
  "gene_name": "Immunoglobulin kappa variable 2D-40",
  "term_label": "Unknown molecular function",
  "gene_symbol": "IGKV2D-40"
}